alpha1-adrenergic receptor activity [GO:0004937] (molecular function) Also known as: alpha1 adrenoceptor Definition: Combining with epinephrine or norepinephrine to initiate a change in cell activity via activation of a G protein, with pharmacological characteristics of alpha1-adrenergic receptors; the activity involves transmitting the signal to the Gq alpha subunit of a heterotrimeric G protein. Sources: GOC:cb, GOC:mah, IUPHAR_GPCR:1274 Relationships: is a type of alpha-adrenergic receptor activity [GO:0004936]